{
  "gene_name": "Rho-related GTP-binding protein RhoF",
  "term_label": "protein kinase binding",
  "gene": "UniProtKB:Q9HBH0",
  "term_id": "GO:0019901",
  "gene_symbol": "RHOF"
}